{
  "gene_symbol": "COQ6",
  "gene_name": "Ubiquinone biosynthesis monooxygenase COQ6, mitochondrial",
  "term_label": "mitochondrion",
  "gene": "UniProtKB:Q9Y2Z9",
  "term_id": "GO:0005739"
}